transducin-mediated opsin signaling pathway [GO:0141190] (biological process) Relationships: is a type of G protein-coupled opsin signaling pathway [GO:0016056] Definition: A G protein-coupled receptor signaling pathway that starts with an opsin molecule being activated by a photon. Opsins include rhodopsin and others visual receptors bind heterotrimeric transducin G proteins upon activation. Activated transducin alpha-subunit activates cGMP phosphodiesterase, which breaks down cGMP. The decrease in cGMP concentration leads to closure of cGMP-gated (CNG) channels, blockage of Na+ influx, and hyperpolarization of photoreceptor plasma membrane, leading to transmission of signal through synapses. The signal is terminated by phosphorylation of the C-terminal tail of rhodopsin by rhodopsin kinase to allow arrestin to bind and block G protein binding. Typical examples are rhabdomeric photoreceptors in the eyes of deuterostomes. Also known as: Gt-mediated opsin signaling pathway, cGMP-mediated opsin signaling pathway, ciliary opsin-mediated signaling pathway, cyclic-GMP-mediated opsin signaling pathway, cyclic-nucleotide-mediated opsin signaling pathway, cGMP-mediated rhodopsin signaling pathway References: PMID:19720651, PMID:36272560, PMID:36499010, PMID:37159291